{
  "gene_symbol": "PRC1",
  "gene_name": "Protein regulator of cytokinesis 1",
  "term_label": "cytoplasm",
  "term_id": "GO:0005737",
  "gene": "UniProtKB:O43663"
}